{
  "gene_name": "Long-chain-fatty-acid--CoA ligase 4",
  "term_label": "long-chain fatty acid metabolic process",
  "term_id": "GO:0001676",
  "gene_symbol": "ACSL4",
  "gene": "UniProtKB:O60488"
}